primary follicle stage [GO:0048160] (BP) Sources: GOC:jid, GOC:mtg_sensu, ISBN:0198542771 Relationships: is a type of GO:0022605 Also known as: mammalian oogenesis stage 3 Definition: The stage in oogenesis when a single layer of cuboidal follicle cells surrounds the oocyte. The oocyte nucleus is large.